{
  "term_id": "GO:0140750",
  "term_label": "nucleosome array spacer activity",
  "gene_symbol": "SMARCA4",
  "gene": "UniProtKB:P51532",
  "gene_name": "Transcription activator BRG1"
}